{
  "term_label": "nucleus",
  "gene_symbol": "ZNF804A",
  "gene_name": "Zinc finger protein 804A",
  "gene": "UniProtKB:Q7Z570",
  "term_id": "GO:0005634"
}